regulation of retrograde protein transport, ER to cytosol [GO:1904152] (biological process) Subtypes: negative regulation of retrograde protein transport, ER to cytosol [GO:1904153], positive regulation of retrograde protein transport, ER to cytosol [GO:1904154] Relationships: is a type of regulation of protein exit from endoplasmic reticulum [GO:0070861]; regulates retrograde protein transport, ER to cytosol [GO:0030970] References: PMID:18555783 Sources: GOC:PARL, GOC:TermGenie, GOC:bf, GO_REF:0000058 Also known as: regulation of protein dislocation from ER, regulation of protein retrotranslocation from ER, regulation of retrograde protein transport, endoplasmic reticulum to cytosol Definition: Any process that modulates the frequency, rate or extent of retrograde protein transport, ER to cytosol.